{
  "term_label": "neuronal cell body",
  "gene_name": "Heat shock protein HSP 90-alpha",
  "gene_symbol": "HSP90AA1",
  "gene": "UniProtKB:P07900",
  "term_id": "GO:0043025"
}